complement component C3d receptor activity [GO:0001860] (molecular function) Relationships: is a type of GO:0004875; has part GO:0001854 Sources: GOC:add, GOC:signaling, ISBN:0781735149 Definition: Combining with the C3d product of the complement cascade and transmitting the signal from one side of the membrane to the other to initiate a change in cell activity.